{
  "term_label": "Unknown molecular function",
  "gene_symbol": "C3orf20",
  "gene": "UniProtKB:Q8ND61",
  "gene_name": "Uncharacterized protein C3orf20",
  "term_id": "UNKNOWN:0001"
}